{
  "gene_name": "LisH domain-containing protein ARMC9",
  "term_id": "GO:0036064",
  "term_label": "ciliary basal body",
  "gene_symbol": "ARMC9",
  "gene": "UniProtKB:Q7Z3E5"
}